{
  "gene_symbol": "TRAJ54",
  "gene": "UniProtKB:A0A075B712",
  "gene_name": "T cell receptor alpha joining 54 (Fragment)",
  "term_label": "Unknown cellular component",
  "term_id": "UNKNOWN:0003"
}